{
  "gene_name": "Protein phosphatase 1 regulatory subunit 32",
  "term_id": "GO:0019902",
  "gene_symbol": "PPP1R32",
  "gene": "UniProtKB:Q7Z5V6",
  "term_label": "phosphatase binding"
}